deoxyribonucleoside metabolic process [GO:0009120] (BP) Relationships: is a type of nucleoside metabolic process [GO:0009116] Also known as: deoxyribonucleoside metabolism Definition: The chemical reactions and pathways involving any one of a family of organic molecules consisting of a purine or pyrimidine base covalently bonded to a sugar deoxyribose (a deoxyribonucleoside). Sources: GOC:jl, ISBN:0140512713 Subtypes: deoxyribonucleoside biosynthetic process [GO:0046120], deoxyribonucleoside catabolic process [GO:0046121], purine deoxyribonucleoside metabolic process [GO:0046122], GO:0046125